{
  "gene_name": "Sphingosine 1-phosphate receptor 1",
  "term_label": "adenylate cyclase-activating G protein-coupled receptor signaling pathway",
  "term_id": "GO:0007189",
  "gene": "UniProtKB:P21453",
  "gene_symbol": "S1PR1"
}